regulation of tridecane biosynthetic process [GO:1900884] (biological process) Also known as: regulation of tridecane anabolism, regulation of tridecane biosynthesis, regulation of tridecane formation, regulation of tridecane synthesis Sources: GOC:TermGenie, GOC:mengo_curators Relationships: is a type of regulation of alkane biosynthetic process [GO:1901577]; regulates tridecane biosynthetic process [GO:1900632] Definition: Any process that modulates the frequency, rate or extent of tridecane biosynthetic process. Subtypes: negative regulation of tridecane biosynthetic process [GO:1900885], positive regulation of tridecane biosynthetic process [GO:1900886]